{
  "gene_name": "Zinc finger protein 277",
  "term_label": "Unknown molecular function",
  "gene": "UniProtKB:Q9NRM2",
  "term_id": "UNKNOWN:0001",
  "gene_symbol": "ZNF277"
}